{
  "gene_name": "Eukaryotic translation initiation factor 4E-binding protein 3",
  "gene": "UniProtKB:O60516",
  "gene_symbol": "EIF4EBP3",
  "term_label": "translation repressor activity",
  "term_id": "GO:0030371"
}